{
  "gene_symbol": "ZNF577",
  "gene": "UniProtKB:Q9BSK1",
  "gene_name": "Zinc finger protein 577",
  "term_id": "GO:0000978",
  "term_label": "RNA polymerase II cis-regulatory region sequence-specific DNA binding"
}